eif4e-cup complex [GO:1990500] (cellular component) Relationships: is a type of translation repressor complex [GO:1903502]; BFO_0000050 GO:0000932 Definition: A protein complex that causes translational repression in Drosophila. Prevents assembly of ribosomes at the mRNA by interfacing with a sequence-specific RNA-binding protein leading to recruitment of the CCR4 complex and consequently, reduction of the mRNA's poly(A) tail length. The complex is also required for dorso-ventral pattern formation in the embryo. Also known as: eukaryotic translation initiation factor 4E-cup complex Note: An example of this is Eif4e in drome (P48598) in PMID:14723848 (inferred from physical interaction). References: PMID:14723848 Sources: GOC:bhm